scyllo-inosamine 4-kinase activity [GO:0050276] (MF) Definition: Catalysis of the reaction: 1-amino-1-deoxy-scyllo-inositol + ATP = 1-amino-1-deoxy-scyllo-inositol 4-phosphate + ADP + 2 H+. Sources: EC:2.7.1.65, RHEA:18605 Also known as: scyllo-inosamine kinase activity, ATP:1-amino-1-deoxy-scyllo-inositol 4-phosphotransferase activity, ATP:inosamine phosphotransferase activity, scyllo-inosamine kinase (phosphorylating) Relationships: is a type of kinase activity [GO:0016301]; is a type of GO:0016773